{
  "gene_name": "Serine_threonine-protein kinase receptor R3",
  "term_label": "BMP receptor complex",
  "gene": "UniProtKB:P37023",
  "term_id": "GO:0070724",
  "gene_symbol": "ACVRL1"
}